{
  "term_id": "UNKNOWN:0003",
  "gene": "UniProtKB:Q96M66",
  "gene_name": "Putative uncharacterized protein FLJ32790",
  "gene_symbol": "Q96M66",
  "term_label": "Unknown cellular component"
}